{
  "gene_name": "Testis-specific Y-encoded protein 3",
  "gene_symbol": "TSPY3",
  "term_label": "chromatin binding",
  "term_id": "GO:0003682",
  "gene": "UniProtKB:P0CV98"
}